{
  "gene": "UniProtKB:Q96SB3",
  "term_id": "GO:0051015",
  "gene_symbol": "PPP1R9B",
  "term_label": "actin filament binding",
  "gene_name": "Neurabin-2"
}